external encapsulating structure organization [GO:0045229] (biological process) Relationships: is a type of cellular component organization [GO:0016043] Definition: A process that is carried out at the cellular level which results in the assembly, arrangement of constituent parts, or disassembly of external structures that lie outside the plasma membrane and surround the entire cell. Also known as: external encapsulating structure organisation, external encapsulating structure organization and biogenesis Sources: GOC:ai, GOC:dph, GOC:jl, GOC:mah Subtypes: GO:0007306, pollen wall assembly [GO:0010208], GO:0030198, cell envelope organization [GO:0043163], capsule organization [GO:0045230], GO:0045231, GO:0045232, exosporium assembly [GO:0070499], cell wall organization [GO:0071555]